response to high population density [GO:0090664] (biological process) Also known as: response to crowding Relationships: is a type of response to stress [GO:0006950]; is a type of multicellular organismal process [GO:0032501] References: PMID:26439857 Sources: GOC:mr Definition: Any process that results in a change in state or activity of a cell or a multicellular organism (in terms of movement, secretion, enzyme production, gene expression, etc.) as a result of a higher than normal number of multicellular organisms living per unit area.